{
  "term_id": "GO:0005096",
  "gene": "UniProtKB:Q9P107",
  "term_label": "GTPase activator activity",
  "gene_name": "GEM-interacting protein",
  "gene_symbol": "GMIP"
}